{
  "term_id": "GO:0007165",
  "term_label": "signal transduction",
  "gene_symbol": "STK11",
  "gene": "UniProtKB:Q15831",
  "gene_name": "Serine_threonine-protein kinase STK11"
}